{
  "term_id": "GO:0006882",
  "gene_symbol": "MT1F",
  "term_label": "intracellular zinc ion homeostasis",
  "gene": "UniProtKB:P04733",
  "gene_name": "Metallothionein-1F"
}